ITPase activity [GO:0103023] (molecular function) Relationships: is_a ribonucleoside triphosphate phosphatase activity [GO:0017111] References: PMID:16216582 Sources: GOC:pz, RHEA:28330 Definition: Catalysis of the reaction: ITP + H2O = IDP + H+ + phosphate.